{
  "term_label": "Unknown molecular function",
  "gene": "UniProtKB:Q96MN9",
  "gene_name": "Zinc finger protein 488",
  "gene_symbol": "ZNF488",
  "term_id": "UNKNOWN:0001"
}